{
  "gene_name": "Cep170-like protein",
  "gene": "UniProtKB:Q96L14",
  "term_id": "UNKNOWN:0001",
  "gene_symbol": "CEP170P1",
  "term_label": "Unknown molecular function"
}